{
  "gene_symbol": "KCNA2",
  "term_id": "GO:0005251",
  "term_label": "delayed rectifier potassium channel activity",
  "gene": "UniProtKB:P16389",
  "gene_name": "Potassium voltage-gated channel subfamily A member 2"
}